{
  "term_id": "GO:0005031",
  "gene_symbol": "TNFRSF1B",
  "gene": "UniProtKB:P20333",
  "gene_name": "Tumor necrosis factor receptor superfamily member 1B",
  "term_label": "tumor necrosis factor receptor activity"
}